{
  "gene_name": "Periostin",
  "term_id": "GO:0031012",
  "gene_symbol": "POSTN",
  "term_label": "extracellular matrix",
  "gene": "UniProtKB:Q15063"
}